negative regulation of regulatory ncRNA-mediated heterochromatin formation [GO:0060906] (biological process) Sources: GOC:dph, GOC:tb Relationships: is a type of GO:0010964; is a type of negative regulation of heterochromatin formation [GO:0031452]; is a type of negative regulation of gene silencing by regulatory ncRNA [GO:0060967]; negatively regulates regulatory ncRNA-mediated heterochromatin formation [GO:0031048] Also known as: negative regulation of RNAi-mediated heterochromatin assembly, negative regulation of ncRNA-mediated heterochromatin formation, negative regulation of heterochromatin assembly by small RNA, negative regulation of small non-coding RNA-mediated heterochromatin formation, negative regulation of chromatin silencing by small RNA Definition: Any process that decreases the frequency, rate or extent of non-coding RNA-mediated heterochromatin formation.